{
  "gene_symbol": "LSP1",
  "gene_name": "Lymphocyte-specific protein 1",
  "gene": "UniProtKB:P33241",
  "term_label": "Unknown molecular function",
  "term_id": "UNKNOWN:0001"
}